{
  "gene_symbol": "IGKV1-9",
  "term_label": "immunoglobulin complex",
  "gene_name": "Immunoglobulin kappa variable 1-9",
  "gene": "UniProtKB:A0A0C4DH69",
  "term_id": "GO:0019814"
}